{
  "gene": "UniProtKB:P01730",
  "term_label": "MHC class II protein complex binding",
  "gene_symbol": "CD4",
  "gene_name": "T-cell surface glycoprotein CD4",
  "term_id": "GO:0023026"
}